{
  "term_id": "UNKNOWN:0002",
  "gene": "UniProtKB:Q9NVU0",
  "gene_symbol": "POLR3E",
  "gene_name": "DNA-directed RNA polymerase III subunit RPC5",
  "term_label": "Unknown biological process"
}